{
  "gene_name": "Ubiquitin conjugation factor E4 B",
  "gene_symbol": "UBE4B",
  "term_id": "GO:0036503",
  "gene": "UniProtKB:O95155",
  "term_label": "ERAD pathway"
}